{
  "gene": "UniProtKB:Q96MK3",
  "term_label": "protein serine/threonine kinase activator activity",
  "gene_symbol": "FAM20A",
  "term_id": "GO:0043539",
  "gene_name": "Pseudokinase FAM20A"
}